IRES-dependent viral translational initiation [GO:0075522] (biological process) Definition: Process by which viral mRNA translation is initiated, where a domain in the 5' untranslated region (UTR) of the viral mRNA called an internal ribosome entry site (IRES) binds the host 43S preinitiation complex, circumventing regular cap-dependent translation initiation. References: PMID:19632368 Sources: GOC:bf, GOC:jl, VZ:867 Relationships: is a type of viral process [GO:0016032]; is part of viral translation [GO:0019081]